regulation of glucosylceramide catabolic process [GO:2000752] (biological process) Definition: Any process that modulates the frequency, rate or extent of glucosylceramide catabolic process. Relationships: is a type of GO:0034248; is a type of regulation of lipid catabolic process [GO:0050994]; is a type of GO:1905038; regulates GO:0006680 Sources: GOC:BHF Subtypes: positive regulation of glucosylceramide catabolic process [GO:2000753] Also known as: regulation of glucosylceramide breakdown, regulation of glucosylceramide catabolism, regulation of glucosylceramide degradation